{
  "term_label": "Unknown molecular function",
  "term_id": "UNKNOWN:0001",
  "gene_symbol": "HCLS1",
  "gene": "UniProtKB:P14317",
  "gene_name": "Hematopoietic lineage cell-specific protein"
}